negative regulation of cell proliferation in dorsal spinal cord [GO:1902832] (BP) Also known as: down regulation of cell proliferation in dorsal spinal cord, down-regulation of cell proliferation in dorsal spinal cord, downregulation of cell proliferation in dorsal spinal cord, inhibition of cell proliferation in dorsal spinal cord References: PMID:21730158 Sources: GOC:TermGenie, GOC:mr, GO_REF:0000058 Definition: Any process that stops, prevents or reduces the frequency, rate or extent of cell proliferation in dorsal spinal cord. Relationships: is a type of regulation of cell proliferation in dorsal spinal cord [GO:0021921]; is a type of GO:2000178; negatively regulates cell proliferation in dorsal spinal cord [GO:0010456]